beta-amyrin 28-monooxygenase activity [GO:0102373] (MF) Relationships: is a type of oxidoreductase activity, acting on paired donors, with incorporation or reduction of molecular oxygen, reduced flavin or flavoprotein as one donor, and incorporation of one atom of oxygen [GO:0016712] Also known as: ursolic aldehyde 28-monooxygenase activity, uvaol dehydrogenase activity Definition: Catalysis of the reaction: beta-amyrin + 3 O2 + 3 reduced [NADPH--hemoprotein reductase] = 4 H+ + 4 H2O + oleanolate + 3 oxidized [NADPH--hemoprotein reductase]. References: PMID:22039103 Sources: RHEA:43068